entrainment of circadian clock [GO:0009649] (biological process) Sources: GOC:jid Definition: The synchronization of a circadian rhythm to environmental time cues such as light. Subtypes: GO:0043153 Also known as: regulation of circadian rhythm phase Relationships: is a type of response to external stimulus [GO:0009605]; is a type of regulation of circadian rhythm [GO:0042752]